{
  "term_id": "GO:0030060",
  "term_label": "L-malate dehydrogenase (NAD+) activity",
  "gene_symbol": "MDH2",
  "gene": "UniProtKB:P40926",
  "gene_name": "Malate dehydrogenase, mitochondrial"
}